barbed-end actin filament capping [GO:0051016] (biological process) Sources: ISBN:071673706X Definition: The binding of a protein or protein complex to the barbed (or plus) end of an actin filament, thus preventing the addition, exchange or removal of further actin subunits. Also known as: barbed-end F-actin capping activity, barbed-end actin capping activity, plus-end F-actin capping activity, plus-end actin filament capping activity Relationships: is a type of actin filament capping [GO:0051693] Regulation: regulated by regulation of barbed-end actin filament capping [GO:2000812]; negatively regulated by GO:2000813; positively regulated by positive regulation of barbed-end actin filament capping [GO:2000814]